{
  "gene": "UniProtKB:Q504Y2",
  "gene_symbol": "PKDCC",
  "term_id": "GO:0004715",
  "gene_name": "Extracellular tyrosine-protein kinase PKDCC",
  "term_label": "non-membrane spanning protein tyrosine kinase activity"
}